{
  "term_label": "synapse",
  "gene_name": "Acetylcholine receptor subunit beta",
  "term_id": "GO:0045202",
  "gene_symbol": "CHRNB1",
  "gene": "UniProtKB:P11230"
}